{
  "term_id": "GO:0005634",
  "gene_symbol": "PABPN1",
  "term_label": "nucleus",
  "gene": "UniProtKB:Q86U42",
  "gene_name": "Polyadenylate-binding protein 2"
}